negative regulation of response to pullulan [GO:1900519] (biological process) Also known as: down regulation of response to pullulan, down-regulation of response to pullulan, downregulation of response to pullulan, inhibition of response to pullulan Sources: GOC:TermGenie, GOC:mengo_curators Relationships: is a type of negative regulation of response to stimulus [GO:0048585]; is a type of regulation of response to pullulan [GO:1900518]; negatively regulates response to pullulan [GO:0044592] Definition: Any process that stops, prevents or reduces the frequency, rate or extent of response to pullulan.